cell adhesion [GO:0007155] (biological process) Relationships: is a type of cellular process [GO:0009987] Subtypes: cell adhesion involved in retrograde extension [GO:0003392], cell-substrate adhesion [GO:0031589], cell adhesion mediated by integrin [GO:0033627], GO:0060519, cell adhesion involved in heart morphogenesis [GO:0061343], cell-cell adhesion [GO:0098609], cell adhesion involved in sprouting angiogenesis [GO:0120078] Sources: GOC:hb, GOC:pf Regulation: negatively regulated by GO:0007162; regulated by regulation of cell adhesion [GO:0030155]; positively regulated by positive regulation of cell adhesion [GO:0045785] Definition: The attachment of a cell, either to another cell or to an underlying substrate such as the extracellular matrix, via cell adhesion molecules. Also known as: cell adhesion molecule activity, single organism cell adhesion